{
  "gene_name": "E3 ubiquitin-protein ligase SH3RF1",
  "term_id": "GO:0046330",
  "gene_symbol": "SH3RF1",
  "gene": "UniProtKB:Q7Z6J0",
  "term_label": "positive regulation of JNK cascade"
}